{
  "term_id": "UNKNOWN:0001",
  "gene_name": "Coiled-coil domain-containing protein 121",
  "gene_symbol": "CCDC121",
  "gene": "UniProtKB:Q6ZUS5",
  "term_label": "Unknown molecular function"
}